{
  "gene_name": "Protocadherin-12",
  "term_id": "GO:0016339",
  "term_label": "calcium-dependent cell-cell adhesion",
  "gene": "UniProtKB:Q9NPG4",
  "gene_symbol": "PCDH12"
}